{
  "gene_name": "Keratin, type I cytoskeletal 10",
  "gene_symbol": "KRT10",
  "gene": "UniProtKB:P13645",
  "term_id": "GO:0045095",
  "term_label": "keratin filament"
}